{
  "gene_name": "Zinc finger protein 664",
  "gene": "UniProtKB:Q8N3J9",
  "term_label": "regulation of DNA-templated transcription",
  "term_id": "GO:0006355",
  "gene_symbol": "ZNF664"
}